respiratory system development [GO:0060541] (biological process) Definition: The progression of the respiratory system over time from its formation to its mature structure. The respiratory system carries out respiratory gaseous exchange. Relationships: is_a system development [GO:0048731] Subtypes: open tracheal system development [GO:0007424] Sources: GOC:dph